{
  "gene_symbol": "TONSL",
  "gene_name": "Tonsoku-like protein",
  "term_label": "double-strand break repair via homologous recombination",
  "gene": "UniProtKB:Q96HA7",
  "term_id": "GO:0000724"
}